{
  "term_id": "GO:0006897",
  "gene": "UniProtKB:Q9UKN7",
  "term_label": "endocytosis",
  "gene_name": "Unconventional myosin-XV",
  "gene_symbol": "MYO15A"
}